{
  "gene_name": "V-type proton ATPase subunit d 1",
  "term_id": "GO:0046961",
  "gene": "UniProtKB:P61421",
  "term_label": "proton-transporting ATPase activity, rotational mechanism",
  "gene_symbol": "ATP6V0D1"
}